{
  "term_id": "GO:0003682",
  "gene": "UniProtKB:P0CV99",
  "gene_symbol": "TSPY4",
  "term_label": "chromatin binding",
  "gene_name": "Testis-specific Y-encoded protein 4"
}